{
  "gene": "UniProtKB:Q6IQ16",
  "gene_symbol": "SPOPL",
  "term_label": "nucleus",
  "term_id": "GO:0005634",
  "gene_name": "Speckle-type POZ protein-like"
}